{
  "term_id": "GO:0071480",
  "gene_name": "Transmembrane protein 109",
  "term_label": "cellular response to gamma radiation",
  "gene_symbol": "TMEM109",
  "gene": "UniProtKB:Q9BVC6"
}